{
  "gene_name": "Homeobox protein Hox-C10",
  "gene_symbol": "HOXC10",
  "term_id": "GO:0000981",
  "gene": "UniProtKB:Q9NYD6",
  "term_label": "DNA-binding transcription factor activity, RNA polymerase II-specific"
}